{
  "term_id": "GO:0006357",
  "gene_name": "Nucleus accumbens-associated protein 1",
  "gene_symbol": "NACC1",
  "gene": "UniProtKB:Q96RE7",
  "term_label": "regulation of transcription by RNA polymerase II"
}